copper ion transport across blood-brain barrier [GO:0097716] (biological process) Definition: The directed movement of copper (Cu) ions passing through the blood-brain barrier. References: PMID:24614235 Sources: GOC:sl Relationships: is a type of copper ion transport [GO:0006825]; is a type of transport across blood-brain barrier [GO:0150104] Also known as: copper ion transport across BBB